sodium:potassium:chloride symporter activity [GO:0008511] (MF) Also known as: sodium/potassium/chloride symporter activity Sources: TC:2.A.30.1.1 Relationships: is a type of potassium:sodium symporter activity [GO:0009674]; is a type of sodium:chloride symporter activity [GO:0015378]; is_a potassium:chloride symporter activity [GO:0015379] Definition: Enables the transfer of a solute or solutes from one side of a membrane to the other according to the reaction: Na+(out) + K+(out) + Cl-(out) = Na+(in) + K+(in) + Cl-(in).